{
  "gene": "UniProtKB:P20336",
  "term_label": "synaptic vesicle membrane",
  "term_id": "GO:0030672",
  "gene_symbol": "RAB3A",
  "gene_name": "Ras-related protein Rab-3A"
}